{
  "gene": "UniProtKB:Q9Y6D0",
  "term_id": "UNKNOWN:0001",
  "gene_symbol": "SELENOK",
  "gene_name": "Selenoprotein K",
  "term_label": "Unknown molecular function"
}